{
  "gene": "UniProtKB:P05000",
  "gene_name": "Interferon omega-1",
  "term_label": "response to exogenous dsRNA",
  "term_id": "GO:0043330",
  "gene_symbol": "IFNW1"
}